 [go#goslim:metagenomics] Note: Metagenomics GO slim